{
  "gene_symbol": "GNPDA1",
  "term_id": "GO:0004342",
  "gene": "UniProtKB:P46926",
  "term_label": "glucosamine-6-phosphate deaminase activity",
  "gene_name": "Glucosamine-6-phosphate isomerase 1"
}